{
  "gene": "UniProtKB:O15547",
  "term_label": "cell junction",
  "term_id": "GO:0030054",
  "gene_name": "P2X purinoceptor 6",
  "gene_symbol": "P2RX6"
}